semi-lunar valve development [GO:1905314] (biological process) References: PMID:19409885 Sources: GOC:BHF, GOC:TermGenie, GOC:rl, GO_REF:0000094 Subtypes: aortic valve development [GO:0003176], pulmonary valve development [GO:0003177] Also known as: semilunar valve development, semilunar valves development Definition: The process whose specific outcome is the progression of a semi-lunar valve over time, from its formation to the mature structure. Relationships: is a type of heart valve development [GO:0003170]